{
  "gene": "UniProtKB:Q9Y5Z7",
  "gene_name": "Host cell factor 2",
  "gene_symbol": "HCFC2",
  "term_label": "chromatin remodeling",
  "term_id": "GO:0006338"
}